{
  "gene_symbol": "AHRR",
  "gene_name": "Aryl hydrocarbon receptor repressor",
  "gene": "UniProtKB:A9YTQ3",
  "term_id": "GO:0000976",
  "term_label": "transcription cis-regulatory region binding"
}